{
  "gene_name": "Paired mesoderm homeobox protein 1",
  "gene": "UniProtKB:P54821",
  "gene_symbol": "PRRX1",
  "term_label": "DNA-binding transcription factor activity, RNA polymerase II-specific",
  "term_id": "GO:0000981"
}